otolith morphogenesis [GO:0032474] (biological process) Relationships: is a type of embryonic morphogenesis [GO:0048598]; is part of inner ear morphogenesis [GO:0042472]; is part of otolith development [GO:0048840] Definition: The process in which the anatomical structures of an otolith are generated and organized. Sources: GOC:dgh